{
  "gene": "UniProtKB:Q70EL3",
  "term_label": "Ras protein signal transduction",
  "term_id": "GO:0007265",
  "gene_symbol": "USP50",
  "gene_name": "Inactive ubiquitin carboxyl-terminal hydrolase 50"
}